{
  "term_label": "regulation of gene expression",
  "term_id": "GO:0010468",
  "gene": "UniProtKB:Q8NI38",
  "gene_name": "NF-kappa-B inhibitor delta",
  "gene_symbol": "NFKBID"
}